{
  "gene_symbol": "ADAM15",
  "gene_name": "Disintegrin and metalloproteinase domain-containing protein 15",
  "term_id": "GO:0045087",
  "term_label": "innate immune response",
  "gene": "UniProtKB:Q13444"
}